{
  "gene_name": "Iroquois-class homeodomain protein IRX-2",
  "gene_symbol": "IRX2",
  "gene": "UniProtKB:Q9BZI1",
  "term_id": "GO:0006357",
  "term_label": "regulation of transcription by RNA polymerase II"
}